{
  "term_label": "pattern recognition receptor activity",
  "gene": "UniProtKB:Q9Y2G2",
  "gene_name": "Caspase recruitment domain-containing protein 8",
  "term_id": "GO:0038187",
  "gene_symbol": "CARD8"
}